{
  "term_label": "signal transduction",
  "gene_name": "Tyrosine-protein phosphatase non-receptor type 9",
  "gene_symbol": "PTPN9",
  "gene": "UniProtKB:P43378",
  "term_id": "GO:0007165"
}